regulation of replicative senescence [GO:1904726] (biological process) Relationships: is a type of regulation of cell cycle process [GO:0010564]; regulates replicative senescence [GO:0090399] References: PMID:23496142 Sources: GOC:BHF, GOC:BHF_miRNA, GOC:TermGenie, GOC:rph, GO_REF:0000058 Definition: Any process that modulates the frequency, rate or extent of replicative senescence. Subtypes: GO:1904727, positive regulation of replicative senescence [GO:1904728]